{
  "gene_name": "Syntaxin-17",
  "gene_symbol": "STX17",
  "gene": "UniProtKB:P56962",
  "term_label": "SNARE binding",
  "term_id": "GO:0000149"
}